regulation of retinoic acid receptor signaling pathway [GO:0048385] (BP) Subtypes: positive regulation of retinoic acid receptor signaling pathway [GO:0048386], negative regulation of retinoic acid receptor signaling pathway [GO:0048387] Definition: Any process that modulates the frequency, rate or extent of retinoic acid receptor signaling pathway activity. Relationships: is a type of regulation of intracellular signal transduction [GO:1902531]; RO_0002211 retinoic acid receptor signaling pathway [GO:0048384] Also known as: regulation of RAR signaling pathway, regulation of retinoic acid receptor signalling pathway Sources: GOC:dgh